{
  "gene_symbol": "EGLN2",
  "term_label": "ferrous iron binding",
  "gene_name": "Prolyl hydroxylase EGLN2",
  "term_id": "GO:0008198",
  "gene": "UniProtKB:Q96KS0"
}